photoreceptor proximal connecting cilium [GO:0120205] (cellular component) Relationships: is a type of cellular anatomical structure [GO:0110165]; is part of photoreceptor connecting cilium [GO:0032391] References: PMID:29899041 Sources: GOC:krc Also known as: PCC, photoreceptor PCC Definition: The proximal region of the photoreceptor connecting cilium is similar to the transition zone of unspecialized primary cilia and houses several major transition zone complexes, including NPHP, MKS, and RPGR.